mitochondrial transmembrane transport [GO:1990542] (biological process) Definition: The process in which a solute is transported from one side of a membrane to the other into, out of or within a mitochondrion. References: PMID:20533899 Relationships: is a type of GO:0006839; is_a transmembrane transport [GO:0055085] Subtypes: carnitine shuttle [GO:0006853], GO:0170036, export from the mitochondrion [GO:0170037], mitochondrial L-ornithine transmembrane transport [GO:1990575]